{
  "term_id": "GO:0009966",
  "term_label": "regulation of signal transduction",
  "gene_symbol": "HPCAL4",
  "gene_name": "Hippocalcin-like protein 4",
  "gene": "UniProtKB:Q9UM19"
}